{
  "term_id": "GO:0006120",
  "term_label": "mitochondrial electron transport, NADH to ubiquinone",
  "gene_name": "NADH dehydrogenase [ubiquinone] iron-sulfur protein 6, mitochondrial",
  "gene_symbol": "NDUFS6",
  "gene": "UniProtKB:O75380"
}